viral portal complex [GO:0046798] (cellular component) Relationships: is a type of protein-containing complex [GO:0032991]; BFO_0000050 viral capsid [GO:0019028] References: PMID:11602732 Definition: A multimeric ring of proteins through which the DNA enters and exits the viral capsid.